serine decarboxylase activity [GO:0102705] (molecular function) Definition: Catalysis of the reaction: H+ + L-serine = ethanolaminium(1+) + carbon dioxide. References: PMID:11461929 Sources: GOC:pz, RHEA:45824 Relationships: is a type of carboxy-lyase activity [GO:0016831]